{
  "gene_symbol": "AGTR1",
  "term_id": "GO:0001596",
  "gene_name": "Type-1 angiotensin II receptor",
  "gene": "UniProtKB:P30556",
  "term_label": "angiotensin type I receptor activity"
}